{
  "gene": "UniProtKB:P15812",
  "term_id": "GO:0005615",
  "gene_name": "T-cell surface glycoprotein CD1e, membrane-associated",
  "term_label": "extracellular space",
  "gene_symbol": "CD1E"
}